{
  "gene": "UniProtKB:Q8WWN9",
  "term_label": "protein-macromolecule adaptor activity",
  "gene_symbol": "IPCEF1",
  "term_id": "GO:0030674",
  "gene_name": "Interactor protein for cytohesin exchange factors 1"
}